{
  "gene_name": "Lysophospholipid acyltransferase 5",
  "term_label": "lysophospholipid acyltransferase activity",
  "term_id": "GO:0071617",
  "gene_symbol": "LPCAT3",
  "gene": "UniProtKB:Q6P1A2"
}